{
  "term_label": "Cul3-RING ubiquitin ligase complex",
  "gene": "UniProtKB:Q9NR64",
  "gene_symbol": "KLHL1",
  "term_id": "GO:0031463",
  "gene_name": "Kelch-like protein 1"
}